{
  "term_label": "Unknown molecular function",
  "gene_name": "BRD4-interacting chromatin-remodeling complex-associated protein-like",
  "gene_symbol": "BICRAL",
  "term_id": "UNKNOWN:0001",
  "gene": "UniProtKB:Q6AI39"
}